{
  "gene_name": "Ribonuclease 8",
  "term_label": "defense response to Gram-positive bacterium",
  "term_id": "GO:0050830",
  "gene": "UniProtKB:Q8TDE3",
  "gene_symbol": "RNASE8"
}